{
  "gene_name": "E3 ubiquitin-protein ligase BRE1A",
  "term_id": "GO:0061630",
  "gene": "UniProtKB:Q5VTR2",
  "term_label": "ubiquitin protein ligase activity",
  "gene_symbol": "RNF20"
}